{
  "gene_symbol": "RGS9",
  "term_label": "G protein-coupled dopamine receptor signaling pathway",
  "term_id": "GO:0007212",
  "gene": "UniProtKB:O75916",
  "gene_name": "Regulator of G-protein signaling 9"
}